{
  "term_label": "potassium ion transmembrane transport",
  "term_id": "GO:0071805",
  "gene_name": "Sodium_hydrogen exchanger 5",
  "gene_symbol": "SLC9A5",
  "gene": "UniProtKB:Q14940"
}